regulation of protein localization to nucleus [GO:1900180] (biological process) Definition: Any process that modulates the frequency, rate or extent of protein localization to nucleus. Sources: GOC:TermGenie Also known as: regulation of protein localisation to nucleus, regulation of protein localization in cell nucleus, regulation of protein localization in nucleus Relationships: is_a regulation of protein localization [GO:0032880]; regulates protein localization to nucleus [GO:0034504] Subtypes: regulation of protein import into nucleus [GO:0042306], negative regulation of protein localization to nucleus [GO:1900181], GO:1900182, regulation of protein localization to nucleolus [GO:1904749], regulation of protein localization to Cajal body [GO:1904869]